{
  "gene_name": "Dipeptidyl aminopeptidase-like protein 6",
  "term_label": "regulation of potassium ion transmembrane transport",
  "gene": "UniProtKB:P42658",
  "gene_symbol": "DPP6",
  "term_id": "GO:1901379"
}